{
  "term_label": "Unknown molecular function",
  "gene_symbol": "MRO",
  "term_id": "UNKNOWN:0001",
  "gene": "UniProtKB:Q9BYG7",
  "gene_name": "Protein maestro"
}